peripheral B cell selection [GO:0002343] (biological process) Relationships: is a type of B cell selection [GO:0002339] Also known as: peripheral B lymphocyte selection, peripheral B-cell selection, peripheral B-lymphocyte selection Subtypes: GO:0002344, peripheral B cell positive selection [GO:0002350], peripheral B cell negative selection [GO:0002356] Sources: GOC:jal Definition: Any B cell selection process that occurs in the periphery.